{
  "term_id": "GO:0061844",
  "gene": "UniProtKB:P58876",
  "term_label": "antimicrobial humoral immune response mediated by antimicrobial peptide",
  "gene_name": "Histone H2B type 1-D",
  "gene_symbol": "H2BC5"
}